monocyte activation [GO:0042117] (biological process) Subtypes: GO:0002280 Definition: The change in morphology and behavior of a monocyte resulting from exposure to a cytokine, chemokine, cellular ligand, or soluble factor. Regulation: negatively regulated by GO:0150102 Relationships: is a type of myeloid leukocyte activation [GO:0002274] Sources: GOC:mgi_curators, ISBN:0781735149